germ cell repulsion [GO:0035233] (biological process) References: PMID:12885551 Definition: The directed movement of a germ cell from their site of production to the gonad, through the repulsion of cells away from a tissue. Relationships: is a type of negative chemotaxis [GO:0050919]; is a type of cell chemotaxis [GO:0060326]; is part of germ cell migration [GO:0008354]